{
  "term_id": "GO:0005634",
  "gene_name": "ATPase family AAA domain-containing protein 2B",
  "term_label": "nucleus",
  "gene_symbol": "ATAD2B",
  "gene": "UniProtKB:Q9ULI0"
}